{
  "gene": "UniProtKB:A0A3B3IRV3",
  "term_id": "UNKNOWN:0001",
  "gene_symbol": "MCTS2",
  "term_label": "Unknown molecular function",
  "gene_name": "Malignant T-cell-amplified sequence 2"
}